{
  "gene": "UniProtKB:Q6UW15",
  "term_id": "GO:0043434",
  "gene_symbol": "REG3G",
  "term_label": "response to peptide hormone",
  "gene_name": "Regenerating islet-derived protein 3-gamma"
}